{
  "term_id": "UNKNOWN:0002",
  "gene_symbol": "TCEAL6",
  "gene_name": "Transcription elongation factor A protein-like 6",
  "gene": "UniProtKB:Q6IPX3",
  "term_label": "Unknown biological process"
}